regulation of rDNA heterochromatin formation [GO:0061187] (BP) Also known as: regulation of chromatin silencing at rDNA, regulation of ribosomal DNA heterochromatin assembly Definition: Any process that modulates the rate, frequency, or extent of rDNA heterochromatin formation. References: PMID:10388812 Relationships: is a type of regulation of heterochromatin formation [GO:0031445]; regulates rDNA heterochromatin formation [GO:0000183] Subtypes: negative regulation of rDNA heterochromatin formation [GO:0061188], positive regulation of rDNA heterochromatin formation [GO:2000749]